{
  "term_id": "GO:0003682",
  "term_label": "chromatin binding",
  "gene": "UniProtKB:P55209",
  "gene_name": "Nucleosome assembly protein 1-like 1",
  "gene_symbol": "NAP1L1"
}